{
  "term_id": "GO:0006357",
  "gene_symbol": "ZNF383",
  "gene_name": "Zinc finger protein 383",
  "gene": "UniProtKB:Q8NA42",
  "term_label": "regulation of transcription by RNA polymerase II"
}